{
  "term_label": "endosomal transport",
  "gene_name": "RalBP1-associated Eps domain-containing protein 2",
  "term_id": "GO:0016197",
  "gene_symbol": "REPS2",
  "gene": "UniProtKB:Q8NFH8"
}